{
  "gene_symbol": "C4orf36",
  "gene": "UniProtKB:Q96KX1",
  "gene_name": "Uncharacterized protein C4orf36",
  "term_label": "Unknown biological process",
  "term_id": "UNKNOWN:0002"
}